maltose synthase activity [GO:0050420] (molecular function) Relationships: is a type of hexosyltransferase activity [GO:0016758] Also known as: alpha-D-glucose-1-phosphate:alpha-D-glucose-1-phosphate 4-alpha-D-glucosyltransferase (dephosphorylating) Sources: EC:2.4.1.139, MetaCyc:MALTOSE-SYNTHASE-RXN Definition: Catalysis of the reaction: 2 alpha-D-glucose 1-phosphate = maltose + 2 phosphate.